S-nitrosoglutathione reductase (NADH) activity [GO:0080007] (molecular function) Definition: Catalysis of the reaction: S-nitrosoglutathione + NADH + H+ = S-(hydroxysulfenamide)glutathione + NAD+. References: PMID:11260719, PMID:27094420, PMID:30795534 Note: S-(hydroxysulfenamide)glutathione (GSNHOH) is an unstable intermediate. At high GSH levels, it is decomposed to glutathione disulfide (GSSG) and hydroxylamine. At low GSH levels, GSNHOH spontaneously converts to glutathione sulfinamid (GSONH2), which can be hydrolyzed to glutathione sulfinic acid (GSOOH) and ammonia. Relationships: is a type of GO:0016616